{
  "term_label": "calcium ion binding",
  "gene": "UniProtKB:P09486",
  "term_id": "GO:0005509",
  "gene_symbol": "SPARC",
  "gene_name": "SPARC"
}